protocadherin-alpha-protocadherin-gamma complex [GO:0071183] (cellular component) Definition: A protein complex that contains two cell adhesion molecules, a protocadherin-alpha and a protocadherin-gamma, and is involved in the regulation of protein localization to the plasma membrane. References: PMID:15347688 Subtypes: protocadherin-alpha-v4-protocadherin-gamma-a1 complex [GO:0071184], protocadherin-alpha-v4-protocadherin-gamma-a3 complex [GO:0071185], protocadherin-alpha-v4-protocadherin-gamma-b2 complex [GO:0071186], protocadherin-alpha-v4-protocadherin-gamma-b4 complex [GO:0071187], protocadherin-alpha-v7-protocadherin-gamma-a1 complex [GO:0071188], protocadherin-alpha-v7-protocadherin-gamma-a3 complex [GO:0071189], protocadherin-alpha-v7-protocadherin-gamma-b2 complex [GO:0071190], GO:0071191 Relationships: is a type of plasma membrane protein complex [GO:0098797]